{
  "term_label": "endoplasmic reticulum",
  "gene": "UniProtKB:Q9NZL4",
  "gene_symbol": "HSPBP1",
  "gene_name": "Hsp70-binding protein 1",
  "term_id": "GO:0005783"
}